{
  "gene": "UniProtKB:A6NN73",
  "term_label": "Golgi organization",
  "term_id": "GO:0007030",
  "gene_symbol": "GOLGA8CP",
  "gene_name": "Golgin subfamily A member 8C"
}